{
  "term_id": "GO:0004816",
  "gene_name": "Asparagine--tRNA ligase, cytoplasmic",
  "term_label": "asparagine-tRNA ligase activity",
  "gene_symbol": "NARS1",
  "gene": "UniProtKB:O43776"
}